{
  "gene": "UniProtKB:Q96RP8",
  "term_id": "GO:0001508",
  "gene_symbol": "KCNA7",
  "term_label": "action potential",
  "gene_name": "Potassium voltage-gated channel subfamily A member 7"
}